{
  "term_label": "immunoglobulin complex",
  "term_id": "GO:0019814",
  "gene": "UniProtKB:A0A0A0MT36",
  "gene_name": "Immunoglobulin kappa variable 6D-21",
  "gene_symbol": "IGKV6D-21"
}